{
  "term_id": "GO:0005737",
  "gene_symbol": "AKAP4",
  "term_label": "cytoplasm",
  "gene": "UniProtKB:Q5JQC9",
  "gene_name": "A-kinase anchor protein 4"
}